lipoteichoic acid binding [GO:0070891] (MF) Definition: Binding to lipoteichoic acid. Relationships: is a type of carbohydrate derivative binding [GO:0097367] References: PMID:14665680 Sources: GOC:add